snRNA transcription by RNA polymerase II [GO:0042795] (biological process) Regulation: regulated by regulation of snRNA transcription by RNA polymerase II [GO:1905380]; negatively regulated by negative regulation of snRNA transcription by RNA polymerase II [GO:1905381]; RO_0002213 by positive regulation of snRNA transcription by RNA polymerase II [GO:1905382] Definition: The synthesis of small nuclear RNA (snRNA) from a DNA template by RNA Polymerase II (Pol II), originating at a Pol II promoter. Relationships: is a type of transcription by RNA polymerase II [GO:0006366]; is a type of snRNA transcription [GO:0009301] Sources: GOC:jl, ISBN:0321000382 Also known as: snRNA transcription from Pol II promoter, snRNA transcription from RNA polymerase II promoter